{
  "gene_name": "Tyrosine 3-monooxygenase",
  "gene": "UniProtKB:P07101",
  "gene_symbol": "TH",
  "term_id": "GO:0043204",
  "term_label": "perikaryon"
}